{
  "term_label": "phosphoglucomutase activity",
  "term_id": "GO:0004614",
  "gene_name": "Phosphoglucomutase-1",
  "gene_symbol": "PGM1",
  "gene": "UniProtKB:P36871"
}